{
  "term_label": "RNA polymerase II cis-regulatory region sequence-specific DNA binding",
  "term_id": "GO:0000978",
  "gene_name": "Transcriptional repressor CTCF",
  "gene_symbol": "CTCF",
  "gene": "UniProtKB:P49711"
}